{
  "term_label": "Unknown biological process",
  "gene_symbol": "LENG8",
  "gene_name": "Leukocyte receptor cluster member 8",
  "gene": "UniProtKB:Q96PV6",
  "term_id": "UNKNOWN:0002"
}